{
  "gene": "UniProtKB:P35240",
  "term_label": "negative regulation of cell population proliferation",
  "term_id": "GO:0008285",
  "gene_name": "Merlin",
  "gene_symbol": "NF2"
}